caveolin-mediated endocytosis [GO:0072584] (biological process) References: PMID:17318224, PMID:18498251, PMID:8970738, PMID:9234965 Sources: GOC:BHF, GOC:mah Subtypes: caveolin-mediated endocytosis of virus by host cell [GO:0075513] Definition: An endocytosis process that begins when material is taken up into plasma membrane caveolae, which then pinch off to form endocytic caveolar carriers. Relationships: is a type of endocytosis [GO:0006897] Regulation: RO_0002211 by GO:2001286; negatively regulated by negative regulation of caveolin-mediated endocytosis [GO:2001287]; RO_0002213 by GO:2001288 Also known as: caveolae-dependent endocytosis, caveolae-mediated endocytosis, caveolin-dependent endocytosis